{
  "gene_name": "Acetylcholine receptor subunit alpha",
  "gene_symbol": "CHRNA1",
  "gene": "UniProtKB:P02708",
  "term_id": "GO:0099171",
  "term_label": "presynaptic modulation of chemical synaptic transmission"
}